{
  "gene": "UniProtKB:P60604",
  "gene_name": "Ubiquitin-conjugating enzyme E2 G2",
  "term_label": "protein polyubiquitination",
  "term_id": "GO:0000209",
  "gene_symbol": "UBE2G2"
}